mycotoxin biosynthetic process [GO:0043386] (biological process) Relationships: is a type of toxin biosynthetic process [GO:0009403]; is a type of mycotoxin metabolic process [GO:0043385] Subtypes: aflatoxin biosynthetic process [GO:0045122], GO:0106110, zearalenone biosynthetic process [GO:0106150], culmorin biosynthetic process [GO:0106210], GO:0140380, GO:0140722, patulin biosynthetic process [GO:0140723], lovastatin biosynthetic process [GO:0140735], ilicicolin H biosynthetic process [GO:0140781], GO:0140783, GO:0140872, GO:0140873, PR-toxin biosynthetic process [GO:0140875], andrastin A biosynthetic process [GO:0140876], mevastatin biosynthetic process [GO:0140877], GO:0140878, conidiogenone biosynthetic process [GO:0140879], GO:0140880, gliotoxin biosynthetic process [GO:2001310] Sources: GOC:jl Definition: The chemical reactions and pathways resulting in the formation of a mycotoxin, any poisonous substance produced by a fungus. Also known as: mycotoxin anabolism, mycotoxin biosynthesis, mycotoxin formation, mycotoxin synthesis